{
  "gene": "UniProtKB:Q8NHW4",
  "gene_name": "C-C motif chemokine 4-like",
  "term_label": "CCR chemokine receptor binding",
  "gene_symbol": "CCL4L1",
  "term_id": "GO:0048020"
}